{
  "gene": "UniProtKB:Q6P9H5",
  "term_id": "GO:0003924",
  "term_label": "GTPase activity",
  "gene_symbol": "GIMAP6",
  "gene_name": "GTPase IMAP family member 6"
}